{
  "gene_symbol": "PPP1R10",
  "term_id": "GO:0004864",
  "gene": "UniProtKB:Q96QC0",
  "gene_name": "Serine_threonine-protein phosphatase 1 regulatory subunit 10",
  "term_label": "protein phosphatase inhibitor activity"
}